{
  "term_label": "ESCRT III complex",
  "gene": "UniProtKB:Q9NZZ3",
  "gene_name": "Charged multivesicular body protein 5",
  "term_id": "GO:0000815",
  "gene_symbol": "CHMP5"
}